presynaptic membrane [GO:0042734] (cellular component) Relationships: is a type of synaptic membrane [GO:0097060]; is part of presynapse [GO:0098793] Sources: GOC:jl, ISBN:0815316194 Definition: A specialized area of membrane of the axon terminal that faces the plasma membrane of the neuron or muscle fiber with which the axon terminal establishes a synaptic junction; many synaptic junctions exhibit structural presynaptic characteristics, such as conical, electron-dense internal protrusions, that distinguish it from the remainder of the axon plasma membrane. Also known as: pre-synaptic membrane, presynaptic plasma membrane